{
  "gene_symbol": "UGT1A3",
  "gene_name": "UDP-glucuronosyltransferase 1A3",
  "gene": "UniProtKB:P35503",
  "term_label": "endoplasmic reticulum",
  "term_id": "GO:0005783"
}